{
  "gene": "UniProtKB:Q14929",
  "gene_symbol": "ZNF169",
  "gene_name": "Zinc finger protein 169",
  "term_label": "RNA polymerase II transcription regulatory region sequence-specific DNA binding",
  "term_id": "GO:0000977"
}